dihydrouracil oxidase activity [GO:0047857] (molecular function) Definition: Catalysis of the reaction: 5,6-dihydrouracil + O2 = H2O2 + uracil. Sources: EC:1.3.3.7, RHEA:12384 Also known as: 5,6-dihydrouracil:oxygen oxidoreductase activity Relationships: is a type of GO:0016634